{
  "gene_name": "AT-rich interactive domain-containing protein 5B",
  "term_label": "regulation of transcription by RNA polymerase II",
  "gene_symbol": "ARID5B",
  "term_id": "GO:0006357",
  "gene": "UniProtKB:Q14865"
}